{
  "term_id": "UNKNOWN:0003",
  "gene_name": "RCC1 domain-containing protein 1",
  "term_label": "Unknown cellular component",
  "gene_symbol": "RCCD1",
  "gene": "UniProtKB:A6NED2"
}